succinate-citramalate CoA-transferase activity [GO:0047370] (molecular function) References: PMID:16547052 Sources: RHEA:38287 Definition: Catalysis of the reaction: S-citramalate + succinyl-CoA = citramalyl-CoA + succinate. Also known as: citramalate coenzyme A-transferase activity, itaconate CoA-transferase activity, succinyl coenzyme A-citramalyl coenzyme A transferase activity, succinyl-CoA:citramalate CoA-transferase activity Relationships: is a type of CoA-transferase activity [GO:0008410]